positive regulation of toluene catabolic process [GO:1901436] (biological process) Relationships: is a type of positive regulation of catabolic process [GO:0009896]; is a type of GO:1901434; RO_0002213 toluene catabolic process [GO:0042203] Definition: Any process that activates or increases the frequency, rate or extent of toluene catabolic process. Also known as: activation of toluene breakdown, activation of toluene catabolism, activation of toluene degradation, positive regulation of toluene breakdown, positive regulation of toluene catabolism, positive regulation of toluene degradation, up regulation of toluene breakdown, up regulation of toluene catabolic process, up regulation of toluene catabolism, up regulation of toluene degradation, up-regulation of toluene breakdown, up-regulation of toluene catabolic process, up-regulation of toluene catabolism, up-regulation of toluene degradation, upregulation of toluene breakdown, upregulation of toluene catabolic process, upregulation of toluene catabolism, upregulation of toluene degradation, activation of toluene catabolic process Sources: GOC:TermGenie, GOC:mengo_curators